{
  "gene_symbol": "DSCR8",
  "term_label": "Unknown cellular component",
  "term_id": "UNKNOWN:0003",
  "gene_name": "Down syndrome critical region protein 8",
  "gene": "UniProtKB:Q96T75"
}